{
  "term_label": "cytokine activity",
  "gene_name": "Putative uncharacterized protein UNQ5830_PRO19650_PRO19816",
  "term_id": "GO:0005125",
  "gene_symbol": "UNQ5830/PRO19650/PRO19816",
  "gene": "UniProtKB:Q6UY13"
}